poly(5-hydroxyvalerate) biosynthetic process [GO:1902919] (biological process) Relationships: is a type of GO:1902921 Also known as: poly(5-hydroxyvalerate) anabolism, poly(5-hydroxyvalerate) biosynthesis, poly(5-hydroxyvalerate) formation, poly(5-hydroxyvalerate) synthesis References: PMID:21705209 Sources: GOC:TermGenie, GOC:mengo_curators, GO_REF:0000068 Definition: The chemical reactions and pathways resulting in the formation of poly(5-hydroxyvalerate).